{
  "gene_symbol": "SLC35C1",
  "term_label": "Golgi apparatus",
  "gene_name": "GDP-fucose transporter 1",
  "gene": "UniProtKB:Q96A29",
  "term_id": "GO:0005794"
}